{
  "gene": "UniProtKB:P47901",
  "term_id": "GO:0045907",
  "gene_symbol": "AVPR1B",
  "term_label": "positive regulation of vasoconstriction",
  "gene_name": "Vasopressin V1b receptor"
}